{
  "term_label": "extracellular matrix organization",
  "gene_name": "A disintegrin and metalloproteinase with thrombospondin motifs 17",
  "term_id": "GO:0030198",
  "gene": "UniProtKB:Q8TE56",
  "gene_symbol": "ADAMTS17"
}